{
  "gene_symbol": "CERS1",
  "gene": "UniProtKB:P27544",
  "term_id": "GO:0005783",
  "gene_name": "Ceramide synthase 1",
  "term_label": "endoplasmic reticulum"
}